{
  "term_id": "GO:0001533",
  "gene": "UniProtKB:P07476",
  "gene_name": "Involucrin",
  "term_label": "cornified envelope",
  "gene_symbol": "IVL"
}